{
  "gene_symbol": "H2AX",
  "term_label": "structural constituent of chromatin",
  "term_id": "GO:0030527",
  "gene_name": "Histone H2AX",
  "gene": "UniProtKB:P16104"
}